{
  "gene_name": "Death domain-associated protein 6",
  "term_id": "GO:0003713",
  "term_label": "transcription coactivator activity",
  "gene": "UniProtKB:Q9UER7",
  "gene_symbol": "DAXX"
}